{
  "gene_symbol": "CAMTA2",
  "term_id": "GO:0006357",
  "gene": "UniProtKB:O94983",
  "term_label": "regulation of transcription by RNA polymerase II",
  "gene_name": "Calmodulin-binding transcription activator 2"
}